{
  "gene_name": "Extracellular sulfatase Sulf-2",
  "term_label": "positive regulation of Wnt signaling pathway",
  "gene": "UniProtKB:Q8IWU5",
  "gene_symbol": "SULF2",
  "term_id": "GO:0030177"
}